L-aspartate:2-oxoglutarate aminotransferase activity [GO:0004069] (molecular function) Also known as: L-aspartate transaminase activity, L-aspartic aminotransferase activity, aspartate aminotransferase activity, aspartate transaminase activity, aspartic acid aminotransferase activity, aspartic aminotransferase activity, aspartyl aminotransferase activity, 2-oxoglutarate-glutamate aminotransferase activity, AAT, AspT, GOT (enzyme), L-aspartate-2-ketoglutarate aminotransferase activity, L-aspartate-2-oxoglutarate aminotransferase activity, L-aspartate-2-oxoglutarate-transaminase activity, L-aspartate-alpha-ketoglutarate transaminase activity, aspartate alpha-ketoglutarate transaminase activity, aspartate-2-oxoglutarate transaminase activity, aspartate:2-oxoglutarate aminotransferase activity, glutamate oxaloacetate transaminase activity, glutamate-oxalacetate aminotransferase activity, glutamate-oxalate transaminase activity, glutamic oxalic transaminase activity, glutamic--aspartic transaminase activity, glutamic--oxaloacetic transaminase activity, glutamic-aspartic aminotransferase activity, glutamic-oxalacetic transaminase activity, oxaloacetate transferase activity, oxaloacetate-aspartate aminotransferase activity, transaminase A activity Sources: EC:2.6.1.1 Definition: Catalysis of the reaction: L-aspartate + 2-oxoglutarate = oxaloacetate + L-glutamate. Relationships: is a type of transaminase activity [GO:0008483] Note: Note that this term has a MetaCyc pathway reference as the pathway only has a single step.